{
  "gene_name": "Structural maintenance of chromosomes protein 5",
  "term_label": "single-stranded DNA binding",
  "gene": "UniProtKB:Q8IY18",
  "gene_symbol": "SMC5",
  "term_id": "GO:0003697"
}